beta-3 adrenergic receptor binding [GO:0031699] (molecular function) Relationships: is a type of adrenergic receptor binding [GO:0031690] Sources: GOC:mah, GOC:nln Definition: Binding to a beta-3 adrenergic receptor. Also known as: beta-3 adrenergic receptor ligand